{
  "gene": "UniProtKB:Q9BXS9",
  "term_label": "sulfate transmembrane transporter activity",
  "term_id": "GO:0015116",
  "gene_name": "Solute carrier family 26 member 6",
  "gene_symbol": "SLC26A6"
}